{
  "gene_name": "Sodium_hydrogen exchanger 9",
  "term_id": "GO:0051453",
  "gene": "UniProtKB:Q8IVB4",
  "term_label": "regulation of intracellular pH",
  "gene_symbol": "SLC9A9"
}